{
  "term_label": "dTMP kinase activity",
  "gene": "UniProtKB:P23919",
  "term_id": "GO:0004798",
  "gene_name": "Thymidylate kinase",
  "gene_symbol": "DTYMK"
}